synaptic vesicle cycle [GO:0099504] (biological process) Relationships: is a type of establishment of localization in cell [GO:0051649]; is a type of GO:0099003; occurs in presynapse [GO:0098793] References: PMID:15217342 Sources: GOC:aruk, GOC:bc Regulation: regulated by regulation of synaptic vesicle cycle [GO:0098693] Definition: A biological process in which synaptic vesicles are loaded with neurotransmitters, move to the active zone, exocytose and are then recycled via endocytosis, ultimately leading to reloading with neurotransmitters.